{
  "gene": "UniProtKB:P15382",
  "term_id": "GO:0015459",
  "gene_name": "Potassium voltage-gated channel subfamily E member 1",
  "gene_symbol": "KCNE1",
  "term_label": "potassium channel regulator activity"
}